regulation of eosinophil chemotaxis [GO:2000422] (biological process) Subtypes: negative regulation of eosinophil chemotaxis [GO:2000423], positive regulation of eosinophil chemotaxis [GO:2000424] Relationships: is a type of regulation of granulocyte chemotaxis [GO:0071622]; is a type of regulation of eosinophil migration [GO:2000416]; regulates eosinophil chemotaxis [GO:0048245] Sources: GOC:obol Definition: Any process that modulates the frequency, rate or extent of eosinophil chemotaxis.